{
  "gene_name": "WD repeat-containing protein 37",
  "term_label": "Unknown cellular component",
  "gene_symbol": "WDR37",
  "term_id": "UNKNOWN:0003",
  "gene": "UniProtKB:Q9Y2I8"
}